aspartate secretion, neurotransmission [GO:0061530] (biological process) Definition: The regulated release of aspartate by a cell in which the aspartate acts as a neurotransmitter. Relationships: is a type of GO:0007269; is a type of aspartate secretion [GO:0061528] Sources: GOC:dph